{
  "gene": "UniProtKB:Q2TAP0",
  "term_label": "Unknown molecular function",
  "term_id": "UNKNOWN:0001",
  "gene_name": "Golgin subfamily A member 7B",
  "gene_symbol": "GOLGA7B"
}